{
  "term_label": "superoxide anion generation",
  "gene": "UniProtKB:P19878",
  "gene_symbol": "NCF2",
  "gene_name": "Neutrophil cytosol factor 2",
  "term_id": "GO:0042554"
}